{
  "gene_name": "Lysosome-associated membrane glycoprotein 5",
  "term_id": "GO:0005765",
  "term_label": "lysosomal membrane",
  "gene": "UniProtKB:Q9UJQ1",
  "gene_symbol": "LAMP5"
}